{
  "term_id": "GO:0005125",
  "gene_symbol": "IFNA21",
  "gene": "UniProtKB:P01568",
  "term_label": "cytokine activity",
  "gene_name": "Interferon alpha-21"
}